{
  "term_label": "R2TP complex",
  "gene_name": "RuvB-like 2",
  "gene_symbol": "RUVBL2",
  "term_id": "GO:0097255",
  "gene": "UniProtKB:Q9Y230"
}